regulation of dendritic cell cytokine production [GO:0002730] (biological process) Relationships: is a type of GO:0002703; is a type of regulation of cytokine production involved in immune response [GO:0002718]; regulates GO:0002371 Definition: Any process that modulates the frequency, rate, or extent of dendritic cell cytokine production. Subtypes: negative regulation of dendritic cell cytokine production [GO:0002731], positive regulation of dendritic cell cytokine production [GO:0002732], regulation of myeloid dendritic cell cytokine production [GO:0002733], GO:0002736 Sources: GOC:add